regulation of cell killing [GO:0031341] (biological process) Definition: Any process that modulates the frequency, rate or extent of cell killing, the process in which a cell brings about the death of another cell, either in the same or a different organism. Relationships: is a type of GO:0050794; regulates cell killing [GO:0001906] Sources: GOC:mah Subtypes: regulation of leukocyte mediated cytotoxicity [GO:0001910], negative regulation of cell killing [GO:0031342], positive regulation of cell killing [GO:0031343], regulation of killing of cells of another organism [GO:0051709], regulation of complement-dependent cytotoxicity [GO:1903659]